regulation of skeletal muscle adaptation [GO:0014733] (biological process) Definition: Any process in which skeletal muscle adapts, with consequent modifications to structural and/or functional phenotypes, in response to a stimulus. Stimuli include contractile activity, loading conditions, substrate supply, and environmental factors. These adaptive events occur in both muscle fibers and associated structures (motoneurons and capillaries), and they involve alterations in regulatory mechanisms, contractile properties and metabolic capacities. Subtypes: GO:0014883, transition between slow and fast fiber [GO:0014886], regulation of skeletal muscle hypertrophy [GO:1904204] Relationships: is a type of GO:0043502; regulates skeletal muscle adaptation [GO:0043501] Sources: GOC:mtg_muscle Also known as: regulation of skeletal muscle plasticity